RNA cytidine insertion [GO:0070708] (biological process) Definition: The modification of an RNA molecule by insertion of a cytidine nucleotide. Sources: GOC:cb, GOC:mah Also known as: RNA C insertion Relationships: is a type of RNA nucleotide insertion [GO:0070705]